detection of diacyl bacterial lipopeptide [GO:0042496] (biological process) Also known as: detection of diacylated bacterial lipoprotein, perception of diacylated bacterial lipopeptide, perception of diacylated bacterial lipoprotein Definition: The series of events in which a diacylated bacterial lipopeptide stimulus is received by a cell and converted into a molecular signal. Diacylated bacterial lipoproteins are lipopeptides of bacterial origin containing a nonprotein moiety consisting of two acyl groups. Relationships: is a type of detection of bacterial lipopeptide [GO:0070340]; is a type of response to diacyl bacterial lipopeptide [GO:0071724] Note: Note that bacterial lipopeptides are derived from bacterial lipoproteins, but the two terms are sometimes used interchangeably in the literature. References: PMID:12077222, PMID:12524386, PMID:2757794 Sources: GOC:add